{
  "gene": "UniProtKB:O95264",
  "gene_symbol": "HTR3B",
  "term_id": "GO:0042391",
  "gene_name": "5-hydroxytryptamine receptor 3B",
  "term_label": "regulation of membrane potential"
}